{
  "gene_symbol": "FAT2",
  "gene": "UniProtKB:Q9NYQ8",
  "term_label": "adherens junction",
  "term_id": "GO:0005912",
  "gene_name": "Protocadherin Fat 2"
}